{
  "gene": "UniProtKB:Q8NF91",
  "gene_name": "Nesprin-1",
  "term_id": "GO:0030017",
  "gene_symbol": "SYNE1",
  "term_label": "sarcomere"
}